{
  "gene": "UniProtKB:Q4ZG55",
  "term_id": "GO:0002009",
  "term_label": "morphogenesis of an epithelium",
  "gene_name": "Protein GREB1",
  "gene_symbol": "GREB1"
}